{
  "gene": "UniProtKB:Q9HAK2",
  "term_label": "RNA polymerase II cis-regulatory region sequence-specific DNA binding",
  "gene_symbol": "EBF2",
  "term_id": "GO:0000978",
  "gene_name": "Transcription factor COE2"
}